endomembrane system organization [GO:0010256] (biological process) Relationships: is a type of cellular component organization [GO:0016043] Definition: A process that is carried out at the cellular level which results in the assembly, arrangement of constituent parts, or disassembly of the endomembrane system. Sources: GOC:mah, GOC:sm Also known as: endomembrane organization, endomembrane system organisation